{
  "term_label": "Unknown molecular function",
  "gene_symbol": "ARMC12",
  "gene_name": "Armadillo repeat-containing protein 12",
  "gene": "UniProtKB:Q5T9G4",
  "term_id": "UNKNOWN:0001"
}